{
  "gene": "UniProtKB:O75147",
  "gene_symbol": "OBSL1",
  "term_id": "UNKNOWN:0001",
  "term_label": "Unknown molecular function",
  "gene_name": "Obscurin-like protein 1"
}